{
  "gene_name": "Platelet glycoprotein 4",
  "term_id": "GO:0006898",
  "gene_symbol": "CD36",
  "gene": "UniProtKB:P16671",
  "term_label": "receptor-mediated endocytosis"
}